gamma-butyrobetaine dioxygenase activity [GO:0008336] (molecular function) Also known as: g-butyrobetaine dioxygenase activity, gamma-butyrobetaine,2-oxoglutarate dioxygenase activity, 4-trimethylammoniobutanoate,2-oxoglutarate:oxygen oxidoreductase (3-hydroxylating), alpha-butyrobetaine hydroxylase activity, butyrobetaine hydroxylase activity, gamma-BBH activity, gamma-butyrobetaine hydroxylase activity Relationships: is a type of 2-oxoglutarate-dependent dioxygenase activity [GO:0016706] Sources: EC:1.14.11.1, RHEA:24028 Definition: Catalysis of the reaction: 2-oxoglutarate + 4-(trimethylammonio)butanoate + O2 = carnitine + CO2 + succinate.